regulation of gamma-aminobutyric acid secretion [GO:0014052] (biological process) Also known as: regulation of GABA secretion Sources: GOC:ef Definition: Any process that modulates the frequency, rate or extent of the regulated release of gamma-aminobutyric acid. Relationships: is a type of regulation of organic acid transport [GO:0032890]; is a type of regulation of secretion [GO:0051046]; is_a GO:0051955; regulates gamma-aminobutyric acid secretion [GO:0014051] Subtypes: negative regulation of gamma-aminobutyric acid secretion [GO:0014053], positive regulation of gamma-aminobutyric acid secretion [GO:0014054]